voluntary skeletal muscle contraction [GO:0003010] (biological process) Sources: GOC:mtg_cardio, GOC:mtg_muscle Definition: A process in which force is generated within voluntary skeletal muscle tissue, resulting in a change in muscle geometry. Force generation involves a chemo-mechanical energy conversion step that is carried out by the actin/myosin complex activity, which generates force through ATP hydrolysis. In the voluntary skeletal muscle, the muscle contraction takes advantage of an ordered sarcomeric structure and it is under voluntary control. Voluntary skeletal muscle is skeletal muscle that is under conscious control. Subtypes: oscillatory muscle contraction [GO:0014703], GO:0014720, twitch skeletal muscle contraction [GO:0014721] Relationships: is a type of skeletal muscle contraction [GO:0003009]